female germline ring canal outer rim [GO:0035182] (cellular component) Note: See also the fly_anatomy.ontology term 'outer nurse cell ring canal rim ; FBbt:00004882'. Definition: An electron opaque backbone of the insect ovarian ring canal that is a part of or adjacent to the plasma membrane. The outer rim is established as the cleavage furrow is arrested, and contains F-actin, anillin, glycoproteins and at least one a protein with a high content of phosphorylated tyrosine residues. References: PMID:12435357, PMID:7925006 Relationships: is a type of cellular anatomical structure [GO:0110165]; is part of extracellular region [GO:0005576]; is part of female germline ring canal [GO:0035324] Also known as: germline ring canal outer rim, nurse cell ring canal outer rim, ovarian ring canal outer rim